{
  "gene_symbol": "BAIAP3",
  "gene_name": "BAI1-associated protein 3",
  "term_id": "GO:0055038",
  "gene": "UniProtKB:O94812",
  "term_label": "recycling endosome membrane"
}